positive regulation of intrinsic apoptotic signaling pathway in response to osmotic stress [GO:1902220] (biological process) References: PMID:14569084 Sources: GOC:BHF, GOC:TermGenie, GOC:mtg_apoptosis, GOC:rl Relationships: is a type of regulation of intrinsic apoptotic signaling pathway in response to osmotic stress [GO:1902218]; is a type of positive regulation of intrinsic apoptotic signaling pathway [GO:2001244]; positively regulates intrinsic apoptotic signaling pathway in response to osmotic stress [GO:0008627] Definition: Any process that activates or increases the frequency, rate or extent of intrinsic apoptotic signaling pathway in response to osmotic stress. Subtypes: positive regulation of intrinsic apoptotic signaling pathway in response to osmotic stress by p53 class mediator [GO:1902240] Also known as: up regulation of intrinsic apoptotic signaling pathway in response to osmotic stress, up-regulation of intrinsic apoptotic signaling pathway in response to osmotic stress, upregulation of intrinsic apoptotic signaling pathway in response to osmotic stress, activation of intrinsic apoptotic signaling pathway in response to osmotic stress